estrogen biosynthetic process [GO:0006703] (biological process) Relationships: is a type of estrogen metabolic process [GO:0008210]; is a type of hormone biosynthetic process [GO:0042446]; is a type of steroid hormone biosynthetic process [GO:0120178] Regulation: regulated by regulation of estrogen biosynthetic process [GO:1904076]; negatively regulated by negative regulation of estrogen biosynthetic process [GO:1904077]; positively regulated by positive regulation of estrogen biosynthetic process [GO:1904078] Also known as: estrogen anabolism, estrogen biosynthesis, estrogen formation, estrogen synthesis, oestrogen biosynthesis, oestrogen biosynthetic process Sources: ISBN:0198506732 Definition: The chemical reactions and pathways resulting in the formation of estrogens, C18 steroid hormones that can stimulate the development of female sexual characteristics. Also found in plants.